retrotrapezoid nucleus development [GO:0061451] (biological process) Sources: GOC:dph Definition: The progression of the retrotrapezoid nucleus (RTN) over time from it's initial formation to its mature state. The retrotrapezoid nucleus is a group of neurons in the rostral medulla, which are responsible regulating respiration. Relationships: is a type of neural nucleus development [GO:0048857]; is part of medulla oblongata development [GO:0021550]